indolebutyric acid metabolic process [GO:0080024] (biological process) Relationships: is_a auxin metabolic process [GO:0009850]; is a type of GO:0032787; is a type of indole-containing compound metabolic process [GO:0042430] Also known as: IBA metabolic process, IBA metabolism, indole-3-butyric acid metabolic process Definition: The chemical reactions and pathways involving indolebutyric acid, a compound that serves as an active or storage form of the hormone indole-3-acetic acid (an auxin) in many plants. References: PMID:18725356